{
  "term_label": "molecular adaptor activity",
  "gene_name": "Small glutamine-rich tetratricopeptide repeat-containing protein alpha",
  "gene_symbol": "SGTA",
  "term_id": "GO:0060090",
  "gene": "UniProtKB:O43765"
}